positive regulation of cellular response to heat [GO:1900036] (biological process) Sources: GOC:TermGenie, GOC:yaf Also known as: activation of cellular response to heat stress, positive regulation of cellular response to heat stress, up regulation of cellular response to heat stress, up-regulation of cellular response to heat stress, upregulation of cellular response to heat stress, activation of cellular response to heat, up regulation of cellular response to heat, up-regulation of cellular response to heat, upregulation of cellular response to heat Definition: Any process that activates or increases the frequency, rate or extent of cellular response to heat. Relationships: is_a positive regulation of cellular process [GO:0048522]; is a type of positive regulation of response to stimulus [GO:0048584]; is a type of regulation of cellular response to heat [GO:1900034]; positively regulates cellular response to heat [GO:0034605]